{
  "term_label": "Unknown biological process",
  "gene_name": "Proteasomal ATPase-associated factor 1",
  "gene": "UniProtKB:Q9BRP4",
  "term_id": "UNKNOWN:0002",
  "gene_symbol": "PAAF1"
}